{
  "term_id": "GO:0007062",
  "gene": "UniProtKB:Q9H4I0",
  "gene_symbol": "RAD21L1",
  "term_label": "sister chromatid cohesion",
  "gene_name": "Double-strand-break repair protein rad21-like protein 1"
}